{
  "gene": "UniProtKB:Q8N6L0",
  "term_id": "GO:0000781",
  "term_label": "chromosome, telomeric region",
  "gene_symbol": "KASH5",
  "gene_name": "Protein KASH5"
}